L-lysine catabolic process to acetyl-CoA [GO:0019474] (biological process) Definition: The chemical reactions and pathways resulting in the breakdown of L-lysine into other compounds, including acetyl-CoA. Subtypes: L-lysine catabolic process to acetyl-CoA via saccharopine [GO:0033512], L-lysine catabolic process to acetyl-CoA via 5-aminopentanamide [GO:0033513], GO:0033514, GO:0033515 Sources: GOC:go_curators Also known as: L-lysine breakdown to acetyl-CoA, L-lysine degradation to acetyl-CoA Relationships: is a type of acetyl-CoA metabolic process [GO:0006084]; is_a L-lysine catabolic process [GO:0019477]; is a type of amide catabolic process [GO:0043605]